{
  "term_label": "Unknown biological process",
  "gene_symbol": "USP11",
  "term_id": "UNKNOWN:0002",
  "gene": "UniProtKB:P51784",
  "gene_name": "Ubiquitin carboxyl-terminal hydrolase 11"
}